synaptic vesicle budding from endosome [GO:0016182] (biological process) Also known as: synaptic vesicle budding involved in synaptic vesicle exocytosis, endosome to synaptic vesicle budding Relationships: is a type of GO:0046907; is_a synaptic vesicle budding [GO:0070142]; is a type of vesicle-mediated transport in synapse [GO:0099003]; is part of synaptic vesicle recycling via endosome [GO:0036466] References: PMID:10099709, PMID:24596248 Sources: GOC:curators Definition: Budding of synaptic vesicles during the formation of constitutive recycling vesicles from early endosomes.